{
  "gene_symbol": "HHIPL2",
  "gene_name": "HHIP-like protein 2",
  "term_id": "UNKNOWN:0003",
  "term_label": "Unknown cellular component",
  "gene": "UniProtKB:Q6UWX4"
}